oxygen-dependent protoporphyrinogen oxidase activity [GO:0004729] (molecular function) Definition: Catalysis of the reaction: 3 O2 + protoporphyrinogen IX = 3 H2O2 + protoporphyrin IX. Relationships: is a type of oxidoreductase activity, acting on the CH-CH group of donors, oxygen as acceptor [GO:0016634]; is a type of GO:0070818 Also known as: protoporphyrinogen-IX:oxygen oxidoreductase activity Sources: RHEA:25576